{
  "term_label": "Rap protein signal transduction",
  "term_id": "GO:0032486",
  "gene_name": "Rap guanine nucleotide exchange factor 3",
  "gene_symbol": "RAPGEF3",
  "gene": "UniProtKB:O95398"
}